alpha-1,3-glucan synthase activity [GO:0047657] (molecular function) Sources: EC:2.4.1.183, MetaCyc:ALPHA-13-GLUCAN-SYNTHASE-RXN Definition: Catalysis of the reaction: UDP-glucose + [alpha-D-glucosyl-(1,3)]n = UDP + [alpha-D-glucosyl-(1,3)]n+1. Relationships: is a type of UDP-glycosyltransferase activity [GO:0008194]; is a type of hexosyltransferase activity [GO:0016758] Also known as: 1,3-alpha-glucan synthase activity, a-1,3-glucan synthase activity, 1,3-alpha-D-glucan synthase activity, UDP-glucose:alpha-D-(1->3)-glucan 3-alpha-D-glucosyltransferase activity, UDPglucose:alpha-D-(1->3)-glucan 3-alpha-D-glucosyltransferase activity, uridine diphosphoglucose-1,3-alpha-glucan glucosyltransferase activity